{
  "gene": "UniProtKB:P05156",
  "term_id": "UNKNOWN:0003",
  "term_label": "Unknown cellular component",
  "gene_symbol": "CFI",
  "gene_name": "Complement factor I"
}